{
  "gene_name": "Transcription factor AP-2-alpha",
  "term_label": "nucleus",
  "gene": "UniProtKB:P05549",
  "term_id": "GO:0005634",
  "gene_symbol": "TFAP2A"
}